{
  "gene": "UniProtKB:Q8NGW1",
  "term_id": "UNKNOWN:0003",
  "gene_name": "Olfactory receptor 6B3",
  "term_label": "Unknown cellular component",
  "gene_symbol": "OR6B3"
}